symbiont-mediated suppression of host translation [GO:0039604] (biological process) Relationships: is_a symbiont-mediated perturbation of host translation [GO:0019057] References: PMID:22046136, PMID:22174690, PMID:32703221 Subtypes: symbiont-mediated inactivation of host ribosome [GO:0141130] Also known as: host translation shutoff, host mRNA cleavage by viral endoribonuclease, host translation shutoff by virus, suppression by virus of host translation, viral host shutoff protein, viral inhibition of cellular protein synthesis, viral shutoff of host protein synthesis Definition: A process in which a symbiont inhibits or disrupts the translation of host mRNA into protein, for example by cleavage of the host mRNAs. The host is defined as the larger of the organisms involved in a symbiotic interaction.